{
  "gene_symbol": "NGEF",
  "term_id": "GO:0032956",
  "gene_name": "Ephexin-1",
  "gene": "UniProtKB:Q8N5V2",
  "term_label": "regulation of actin cytoskeleton organization"
}